{
  "term_id": "UNKNOWN:0003",
  "gene_name": "Zinc finger protein 41",
  "term_label": "Unknown cellular component",
  "gene": "UniProtKB:P51814",
  "gene_symbol": "ZNF41"
}